{
  "gene_symbol": "CARM1",
  "gene_name": "Histone-arginine methyltransferase CARM1",
  "term_label": "chromatin remodeling",
  "gene": "UniProtKB:Q86X55",
  "term_id": "GO:0006338"
}